maintenance of rDNA [GO:0043007] (biological process) Subtypes: replication fork arrest at rDNA repeats [GO:0031582], GO:0045458 Relationships: is a type of maintenance of DNA repeat elements [GO:0043570] References: PMID:14528010 Sources: GOC:vw Definition: Any process involved in sustaining the fidelity and copy number of rDNA repeats. Also known as: rDNA maintenance, ribosomal DNA maintenance